{
  "term_label": "PeBoW complex",
  "gene": "UniProtKB:Q9GZL7",
  "gene_symbol": "WDR12",
  "gene_name": "Ribosome biogenesis protein WDR12",
  "term_id": "GO:0070545"
}